{
  "gene_symbol": "MMP17",
  "term_id": "GO:0005615",
  "term_label": "extracellular space",
  "gene": "UniProtKB:Q9ULZ9",
  "gene_name": "Matrix metalloproteinase-17"
}